{
  "term_label": "cell-cell signaling",
  "gene_name": "Alpha-1B adrenergic receptor",
  "gene_symbol": "ADRA1B",
  "gene": "UniProtKB:P35368",
  "term_id": "GO:0007267"
}